{
  "gene_name": "Zinc finger protein 181",
  "gene_symbol": "ZNF181",
  "term_id": "GO:0006357",
  "term_label": "regulation of transcription by RNA polymerase II",
  "gene": "UniProtKB:Q2M3W8"
}